{
  "gene": "UniProtKB:Q8WWV3",
  "term_label": "ubiquinone biosynthetic process",
  "term_id": "GO:0006744",
  "gene_symbol": "RTN4IP1",
  "gene_name": "Reticulon-4-interacting protein 1, mitochondrial"
}